{
  "gene_symbol": "TOMM6",
  "term_id": "UNKNOWN:0002",
  "term_label": "Unknown biological process",
  "gene_name": "Mitochondrial import receptor subunit TOM6 homolog",
  "gene": "UniProtKB:Q96B49"
}